{
  "gene_name": "High mobility group nucleosome-binding domain-containing protein 5",
  "gene_symbol": "HMGN5",
  "term_label": "Unknown cellular component",
  "gene": "UniProtKB:P82970",
  "term_id": "UNKNOWN:0003"
}